{
  "term_id": "GO:0061061",
  "gene_name": "PDZ and LIM domain protein 5",
  "gene_symbol": "PDLIM5",
  "gene": "UniProtKB:Q96HC4",
  "term_label": "muscle structure development"
}